extrinsic component of dense core granule membrane [GO:0098922] (cellular component) Sources: GOC:dos Definition: The component of the dense core granule membrane consisting of gene products and protein complexes that are loosely bound to one of its surfaces, but not integrated into the hydrophobic region. Subtypes: GO:0098674 Relationships: is a type of extrinsic component of organelle membrane [GO:0031312]; is part of dense core granule membrane [GO:0032127]